negative regulation of cell integrity MAPK cascade [GO:1903138] (biological process) Relationships: is a type of GO:0032873; is a type of regulation of cell integrity MAPK cascade [GO:1903137]; negatively regulates cell integrity MAPK cascade [GO:0000196] Also known as: negative regulation of cell integrity MAPK pathway, inhibition of Mpk1 cascade, inhibition of Pmk1 mitogen-activated protein kinase (MAPK) cell integrity pathway, inhibition of cell wall biogenesis, MAPKKK cascade, negative regulation of MAPK cascade involved in cell wall biogenesis, negative regulation of Mpk1 cascade, negative regulation of PMK1-MAPK signal transduction pathway, negative regulation of Pmk1 MAPK cell integrity signaling, negative regulation of cell wall integrity MAPK cascade Sources: GOC:vw Definition: Any process that stops, prevents or reduces the frequency, rate or extent of a cell integrity MAPK cascade.